{
  "term_id": "UNKNOWN:0002",
  "term_label": "Unknown biological process",
  "gene_symbol": "MYOZ3",
  "gene_name": "Myozenin-3",
  "gene": "UniProtKB:Q8TDC0"
}